glycerol-1-phosphate dehydrogenase (NADP+) activity [GO:0106358] (molecular function) Relationships: is a type of glycerol-1-phosphate dehydrogenase [NAD(P)+] activity [GO:0050492] Definition: Catalysis of the reaction: NADP+ + sn-glycerol 1-phosphate = dihydroxyacetone phosphate + H+ + NADPH. Sources: RHEA:21416 Also known as: glycerol-1-phosphate dehydrogenase [NADP+] activity